{
  "gene_symbol": "SPACA1",
  "gene_name": "Sperm acrosome membrane-associated protein 1",
  "gene": "UniProtKB:Q9HBV2",
  "term_id": "GO:0001675",
  "term_label": "acrosome assembly"
}